{
  "term_id": "GO:2001199",
  "term_label": "negative regulation of dendritic cell differentiation",
  "gene": "UniProtKB:Q96HP8",
  "gene_symbol": "TMEM176A",
  "gene_name": "Transmembrane protein 176A"
}